{
  "gene": "UniProtKB:Q0VD86",
  "term_id": "GO:0005737",
  "term_label": "cytoplasm",
  "gene_symbol": "INCA1",
  "gene_name": "Protein INCA1"
}